{
  "term_id": "UNKNOWN:0003",
  "gene": "UniProtKB:A0A8I5QJV6",
  "term_label": "Unknown cellular component",
  "gene_symbol": "A0A8I5QJV6",
  "gene_name": "Uncharacterized protein"
}